{
  "gene_name": "Signal transducer and activator of transcription 3",
  "term_id": "GO:0042127",
  "term_label": "regulation of cell population proliferation",
  "gene": "UniProtKB:P40763",
  "gene_symbol": "STAT3"
}